{
  "gene_name": "Ras-related GTP-binding protein A",
  "gene_symbol": "RRAGA",
  "gene": "UniProtKB:Q7L523",
  "term_label": "positive regulation of TORC1 signaling",
  "term_id": "GO:1904263"
}